GDP phosphatase activity [GO:0004382] (molecular function) Also known as: guanosine diphosphatase activity, guanosine-diphosphatase activity, GDP diphosphatase activity, GDP phosphohydrolase activity, GDPase activity, guanosine 5'-diphosphatase activity Relationships: is a type of nucleoside diphosphate phosphatase activity [GO:0017110] References: PMID:2989286 Sources: RHEA:22156 Definition: Catalysis of the reaction: GDP + H2O = GMP + phosphate.